{
  "gene_symbol": "SORCS1",
  "gene_name": "VPS10 domain-containing receptor SorCS1",
  "term_id": "GO:0005794",
  "gene": "UniProtKB:Q8WY21",
  "term_label": "Golgi apparatus"
}